thylakoid membrane disassembly [GO:0010547] (biological process) Relationships: is a type of thylakoid membrane organization [GO:0010027]; is a type of membrane disassembly [GO:0030397] Also known as: thylakoid membrane degradation Definition: The controlled breakdown of the thylakoid membrane in the context of a normal process. References: PMID:17416733 Sources: GOC:dph, GOC:tb Regulation: regulated by regulation of thylakoid membrane disassembly [GO:0010548]